pyrophosphate-dependent phosphofructokinase complex, beta-subunit complex [GO:0010318] (cellular component) References: PMID:2170409 Definition: Refers to the beta subunit of the heterodimeric complex that possesses pyrophosphate-dependent phosphofructokinase activity. Also known as: PFK complex, beta-subunit Relationships: is a type of catalytic complex [GO:1902494]; is part of pyrophosphate-dependent phosphofructokinase complex [GO:0010316]